{
  "gene": "UniProtKB:P02818",
  "term_id": "GO:0008147",
  "gene_symbol": "BGLAP",
  "term_label": "structural constituent of bone",
  "gene_name": "Osteocalcin"
}